{
  "term_id": "UNKNOWN:0001",
  "gene_symbol": "RIF1",
  "gene_name": "Telomere-associated protein RIF1",
  "term_label": "Unknown molecular function",
  "gene": "UniProtKB:Q5UIP0"
}